{
  "gene": "UniProtKB:Q96PQ1",
  "gene_name": "Sialic acid-binding Ig-like lectin 12",
  "gene_symbol": "SIGLEC12",
  "term_id": "GO:0005886",
  "term_label": "plasma membrane"
}